positive regulation of chondrocyte hypertrophy [GO:1903043] (biological process) Definition: Any process that activates or increases the frequency, rate or extent of chondrocyte hypertrophy. References: PMID:23928032 Sources: GOC:TermGenie, GOC:mr, GO_REF:0000058 Also known as: up regulation of chondrocyte hypertrophy, up-regulation of chondrocyte hypertrophy, upregulation of chondrocyte hypertrophy, activation of chondrocyte hypertrophy Relationships: is a type of positive regulation of cell growth [GO:0030307]; is a type of positive regulation of developmental growth [GO:0048639]; is a type of GO:1902761; is a type of GO:1903041; positively regulates chondrocyte hypertrophy [GO:0003415]